positive regulation of postsynaptic cytosolic calcium concentration [GO:0099588] (biological process) Definition: Any process that increases the concentration of calcium ions in the postsynaptic cytosol. Sources: GOC:dos Relationships: is a type of GO:0007204; occurs in postsynapse [GO:0098794]